{
  "term_label": "basolateral plasma membrane",
  "gene": "UniProtKB:P41440",
  "gene_symbol": "SLC19A1",
  "term_id": "GO:0016323",
  "gene_name": "Reduced folate transporter"
}